{
  "gene_name": "Solute carrier family 22 member 13",
  "term_label": "Unknown molecular function",
  "gene_symbol": "SLC22A13",
  "gene": "UniProtKB:Q9Y226",
  "term_id": "UNKNOWN:0001"
}